positive regulation of protein deubiquitination [GO:1903003] (biological process) References: PMID:22970133 Sources: GOC:PARL, GOC:TermGenie, GOC:bf, GO_REF:0000058 Definition: Any process that activates or increases the frequency, rate or extent of protein deubiquitination. Relationships: is a type of regulation of protein deubiquitination [GO:0090085]; is a type of GO:1903322; positively regulates GO:0016579 Also known as: positive regulation of deubiquitination, positive regulation of protein deubiquitinylation, positive regulation of protein deubiquitylation, up regulation of deubiquitination, up regulation of protein deubiquitination, up regulation of protein deubiquitinylation, up regulation of protein deubiquitylation, up-regulation of deubiquitination, up-regulation of protein deubiquitination, up-regulation of protein deubiquitinylation, up-regulation of protein deubiquitylation, upregulation of deubiquitination, upregulation of protein deubiquitination, upregulation of protein deubiquitinylation, upregulation of protein deubiquitylation, activation of deubiquitination, activation of protein deubiquitination, activation of protein deubiquitinylation, activation of protein deubiquitylation Subtypes: positive regulation of protein K63-linked deubiquitination [GO:1903006]